{
  "gene": "UniProtKB:O94776",
  "term_id": "GO:0005654",
  "gene_symbol": "MTA2",
  "term_label": "nucleoplasm",
  "gene_name": "Metastasis-associated protein MTA2"
}